{
  "gene_symbol": "HNRNPCL4",
  "gene_name": "Heterogeneous nuclear ribonucleoprotein C-like 4",
  "gene": "UniProtKB:P0DMR1",
  "term_label": "nucleus",
  "term_id": "GO:0005634"
}